{
  "gene_symbol": "TRAV24",
  "term_id": "UNKNOWN:0003",
  "term_label": "Unknown cellular component",
  "gene": "UniProtKB:A0A0B4J272",
  "gene_name": "T cell receptor alpha variable 24"
}